{
  "term_label": "dendrite",
  "gene_name": "Homer protein homolog 1",
  "term_id": "GO:0030425",
  "gene_symbol": "HOMER1",
  "gene": "UniProtKB:Q86YM7"
}